{
  "gene_symbol": "A0A2R8YCY7",
  "gene": "UniProtKB:A0A2R8YCY7",
  "gene_name": "Immunoglobulin subtype domain-containing protein",
  "term_id": "GO:0140375",
  "term_label": "immune receptor activity"
}